negative regulation of viral transcription [GO:0032897] (BP) Relationships: is a type of regulation of viral transcription [GO:0046782]; is a type of GO:0048525; negatively regulates viral transcription [GO:0019083] Definition: Any process that stops, prevents, or reduces the frequency, rate or extent of viral transcription. Also known as: down regulation of viral transcription, down-regulation of viral transcription, downregulation of viral transcription, inhibition of viral transcription Sources: GOC:mah